{
  "term_label": "Unknown molecular function",
  "gene_symbol": "AKAP12",
  "gene": "UniProtKB:Q02952",
  "gene_name": "A-kinase anchor protein 12",
  "term_id": "UNKNOWN:0001"
}